{
  "gene": "UniProtKB:Q8IWU2",
  "term_label": "protein kinase activity",
  "gene_symbol": "LMTK2",
  "gene_name": "Serine_threonine-protein kinase LMTK2",
  "term_id": "GO:0004672"
}